{
  "gene_symbol": "STN1",
  "term_label": "CST complex",
  "gene_name": "CST complex subunit STN1",
  "term_id": "GO:1990879",
  "gene": "UniProtKB:Q9H668"
}